{
  "gene_name": "C-X-C motif chemokine 17",
  "gene_symbol": "CXCL17",
  "gene": "UniProtKB:Q6UXB2",
  "term_label": "Unknown molecular function",
  "term_id": "UNKNOWN:0001"
}